{
  "gene_name": "Putative ankyrin repeat domain-containing protein 20A12 pseudogene",
  "term_label": "Unknown biological process",
  "gene_symbol": "ANKRD20A12P",
  "term_id": "UNKNOWN:0002",
  "gene": "UniProtKB:Q8NF67"
}